{
  "gene": "UniProtKB:Q8NF99",
  "gene_name": "Zinc finger protein 397",
  "gene_symbol": "ZNF397",
  "term_id": "GO:0006357",
  "term_label": "regulation of transcription by RNA polymerase II"
}